{
  "term_id": "UNKNOWN:0003",
  "gene_symbol": "ACSF2",
  "term_label": "Unknown cellular component",
  "gene": "UniProtKB:Q96CM8",
  "gene_name": "Medium-chain acyl-CoA ligase ACSF2, mitochondrial"
}